negative regulation of cardiac myofibril assembly [GO:1905305] (biological process) Definition: Any process that stops, prevents or reduces the frequency, rate or extent of cardiac myofibril assembly. Also known as: down regulation of cardiac myofibril assembly, down regulation of cardiac myofibril development, down regulation of cardiac myofibril morphogenesis, down-regulation of cardiac myofibril assembly, down-regulation of cardiac myofibril development, down-regulation of cardiac myofibril morphogenesis, downregulation of cardiac myofibril assembly, downregulation of cardiac myofibril development, downregulation of cardiac myofibril morphogenesis, negative regulation of cardiac myofibril development, negative regulation of cardiac myofibril morphogenesis, inhibition of cardiac myofibril assembly, inhibition of cardiac myofibril development, inhibition of cardiac myofibril morphogenesis, down regulation of heart myofibril assembly, down-regulation of heart myofibril assembly, downregulation of heart myofibril assembly, inhibition of heart myofibril assembly, negative regulation of heart myofibril assembly Relationships: is a type of GO:0051494; is a type of negative regulation of organelle assembly [GO:1902116]; is a type of negative regulation of supramolecular fiber organization [GO:1902904]; is_a regulation of cardiac myofibril assembly [GO:1905304]; is a type of negative regulation of cardiac muscle cell differentiation [GO:2000726]; negatively regulates cardiac myofibril assembly [GO:0055003] References: PMID:16151019 Sources: GOC:BHF, GOC:TermGenie, GOC:rl, GO_REF:0000058